regulation of floral organ abscission by signal transduction [GO:0060863] (biological process) Relationships: is a type of signal transduction [GO:0007165]; is a type of regulation of floral organ abscission [GO:0060860] Definition: The cascade of processes by which a signal interacts with a receptor, causing a change in the level or activity of a second messenger or other downstream target, and ultimately modulating the rate, or extent of floral organ abscission. Sources: GOC:dph, GOC:sdb_2009, GOC:tb